negative regulation of photomorphogenesis [GO:0010100] (biological process) Sources: GOC:tb Definition: Any process that stops, reduces or prevents photomorphogenesis. Relationships: is a type of GO:0010099; is a type of GO:0048581; is a type of negative regulation of response to stimulus [GO:0048585]; negatively regulates photomorphogenesis [GO:0009640] Also known as: down regulation of photomorphogenesis, down-regulation of photomorphogenesis, downregulation of photomorphogenesis, inhibition of photomorphogenesis